{
  "term_id": "GO:0000146",
  "gene_symbol": "MYO1F",
  "gene": "UniProtKB:O00160",
  "term_label": "microfilament motor activity",
  "gene_name": "Unconventional myosin-If"
}